{
  "gene": "UniProtKB:P50542",
  "term_label": "protein import into peroxisome matrix, docking",
  "gene_name": "Peroxisomal targeting signal 1 receptor",
  "term_id": "GO:0016560",
  "gene_symbol": "PEX5"
}